{
  "gene_symbol": "MBL2",
  "term_id": "GO:0043129",
  "gene_name": "Mannose-binding protein C",
  "gene": "UniProtKB:P11226",
  "term_label": "surfactant homeostasis"
}